{
  "term_id": "GO:0030071",
  "term_label": "regulation of mitotic metaphase/anaphase transition",
  "gene_name": "Serine_threonine-protein kinase Nek6",
  "gene_symbol": "NEK6",
  "gene": "UniProtKB:Q9HC98"
}